{
  "term_id": "GO:0000151",
  "gene": "UniProtKB:Q96JP0",
  "gene_name": "Protein fem-1 homolog C",
  "gene_symbol": "FEM1C",
  "term_label": "ubiquitin ligase complex"
}